dibenzothiophene catabolic process [GO:0018896] (biological process) Definition: The chemical reactions and pathways resulting in the breakdown of dibenzothiophene, a substance composed of two benzene rings linked by one sulfide bond and one carbon-carbon bond. Also known as: dibenzothiophene breakdown, dibenzothiophene catabolism, dibenzothiophene degradation Sources: GOC:ai Relationships: is a type of xenobiotic catabolic process [GO:0042178]; is a type of sulfur compound catabolic process [GO:0044273]